{
  "gene": "UniProtKB:Q9BQ69",
  "gene_name": "ADP-ribose glycohydrolase MACROD1",
  "gene_symbol": "MACROD1",
  "term_label": "DNA damage response",
  "term_id": "GO:0006974"
}